 [oboInOwl#default-namespace]